dCMP phosphorylation [GO:0061567] (BP) References: PMID:23416111 Sources: GOC:dph Relationships: is a type of GO:0046940 Definition: The process of introducing a phosphate group into dCMP, deoxycytidine monophosphate, to produce dCDP. Addition of two phosphate groups produces dCTP.